CoA-glutathione reductase (NADPH) activity [GO:0050452] (molecular function) Relationships: is a type of oxidoreductase activity, acting on a sulfur group of donors, NAD(P) as acceptor [GO:0016668] Definition: Catalysis of the reaction: CoA + glutathione + NADP+ = CoA-glutathione + NADPH + H+. Sources: RHEA:14617 Also known as: CoA-glutathione reductase activity, coenzyme A disulfide-glutathione reductase activity, coenzyme A glutathione disulfide reductase activity, CoA-glutathione reductase (NADP) activity, NADPH-dependent coenzyme A-SS-glutathione reductase activity, NADPH:CoA-glutathione oxidoreductase activity, glutathione:NADP+ oxidoreductase (CoA-acylating)